{
  "gene_name": "Complement factor H",
  "gene": "UniProtKB:P08603",
  "gene_symbol": "CFH",
  "term_label": "extracellular space",
  "term_id": "GO:0005615"
}